{
  "term_id": "UNKNOWN:0001",
  "gene_name": "Protein RD3-like",
  "gene_symbol": "RD3L",
  "term_label": "Unknown molecular function",
  "gene": "UniProtKB:P0DJH9"
}